{
  "gene_name": "Rhomboid-related protein 1",
  "term_label": "serine-type endopeptidase activity",
  "gene_symbol": "RHBDL1",
  "gene": "UniProtKB:O75783",
  "term_id": "GO:0004252"
}